{
  "term_label": "RNA polymerase II transcription regulatory region sequence-specific DNA binding",
  "term_id": "GO:0000977",
  "gene_symbol": "BARX2",
  "gene_name": "Homeobox protein BarH-like 2",
  "gene": "UniProtKB:Q9UMQ3"
}